{
  "gene_name": "Phosphatidylinositol 4,5-bisphosphate 3-kinase catalytic subunit alpha isoform",
  "gene_symbol": "PIK3CA",
  "gene": "UniProtKB:P42336",
  "term_label": "phosphatidylinositol-3-phosphate biosynthetic process",
  "term_id": "GO:0036092"
}